{
  "gene_name": "RING finger protein 17",
  "gene_symbol": "RNF17",
  "gene": "UniProtKB:Q9BXT8",
  "term_id": "UNKNOWN:0003",
  "term_label": "Unknown cellular component"
}